{
  "gene_name": "Long-chain fatty acid transport protein 4",
  "gene": "UniProtKB:Q6P1M0",
  "gene_symbol": "SLC27A4",
  "term_id": "GO:0005324",
  "term_label": "long-chain fatty acid transmembrane transporter activity"
}